{
  "term_label": "Unknown biological process",
  "gene_name": "Protein FAM229A",
  "gene": "UniProtKB:H3BQW9",
  "term_id": "UNKNOWN:0002",
  "gene_symbol": "FAM229A"
}